{
  "gene_name": "NAD-dependent protein deacetylase sirtuin-1",
  "term_label": "transcription corepressor activity",
  "gene_symbol": "SIRT1",
  "term_id": "GO:0003714",
  "gene": "UniProtKB:Q96EB6"
}